protein histidine tele-kinase activity [GO:0008257] (molecular function) Also known as: protein-histidine tele-kinase activity, ATP:protein-L-histidine N-tele-phosphotransferase activity, ATP:protein-L-histidine Ntau-phosphotransferase activity Relationships: is_a protein histidine kinase activity [GO:0004673] Definition: Catalysis of the reaction: ATP + protein L-histidine = ADP + protein N(tau)-phospho-L-histidine. Sources: EC:2.7.13.2